{
  "gene": "UniProtKB:P54707",
  "gene_name": "Potassium-transporting ATPase alpha chain 2",
  "gene_symbol": "ATP12A",
  "term_label": "potassium ion import across plasma membrane",
  "term_id": "GO:1990573"
}